{
  "gene_symbol": "RASL12",
  "term_id": "GO:0003924",
  "term_label": "GTPase activity",
  "gene": "UniProtKB:Q9NYN1",
  "gene_name": "Ras-like protein family member 12"
}